{
  "gene_symbol": "USP29",
  "gene": "UniProtKB:Q9HBJ7",
  "term_label": "regulation of protein stability",
  "gene_name": "Ubiquitin carboxyl-terminal hydrolase 29",
  "term_id": "GO:0031647"
}